{
  "term_label": "rRNA processing",
  "gene_name": "Cell growth-regulating nucleolar protein",
  "gene": "UniProtKB:Q9NX58",
  "term_id": "GO:0006364",
  "gene_symbol": "LYAR"
}